{
  "gene_symbol": "ARHGAP27",
  "term_label": "small GTPase-mediated signal transduction",
  "term_id": "GO:0007264",
  "gene_name": "Rho GTPase-activating protein 27",
  "gene": "UniProtKB:Q6ZUM4"
}